Kelch-containing formin regulatory complex [GO:1990615] (cellular component) References: PMID:24828508 Definition: A protein complex that regulates actin cable formation, polarized cell growth, and cytokinesis in a formin-dependent manner. In S. cerevisiae the complex is composed of Bud14p and two Kelch family proteins, Kel1p and Kel2p. Relationships: is_a protein-containing complex [GO:0032991] Also known as: KFRC complex, Bud14-Kel1-Kel2 complex